{
  "gene_name": "Retinoic acid early transcript 1E",
  "gene": "UniProtKB:Q8TD07",
  "term_label": "extracellular space",
  "gene_symbol": "RAET1E",
  "term_id": "GO:0005615"
}